{
  "gene": "UniProtKB:Q96LR5",
  "term_id": "GO:0070534",
  "term_label": "protein K63-linked ubiquitination",
  "gene_symbol": "UBE2E2",
  "gene_name": "Ubiquitin-conjugating enzyme E2 E2"
}